{
  "term_label": "nucleus",
  "term_id": "GO:0005634",
  "gene": "UniProtKB:Q6N021",
  "gene_name": "Methylcytosine dioxygenase TET2",
  "gene_symbol": "TET2"
}